root meristem growth [GO:0010449] (biological process) Definition: The increase in size or mass of a root meristem, a population of undifferentiated cells in a plant root which maintains a continuous balance between the production of stem cells and the incorporation of their derivatives into the growth of the root. Sources: GOC:tb Relationships: is a type of meristem growth [GO:0035266]; is part of root development [GO:0048364] Regulation: regulated by GO:0010082